{
  "gene": "UniProtKB:Q96A72",
  "gene_name": "Protein mago nashi homolog 2",
  "term_label": "exon-exon junction complex",
  "term_id": "GO:0035145",
  "gene_symbol": "MAGOHB"
}